{
  "gene": "UniProtKB:Q16821",
  "term_id": "GO:2001069",
  "gene_symbol": "PPP1R3A",
  "gene_name": "Protein phosphatase 1 regulatory subunit 3A",
  "term_label": "glycogen binding"
}